{
  "gene_name": "Band 4.1-like protein 4B",
  "gene": "UniProtKB:Q9H329",
  "gene_symbol": "EPB41L4B",
  "term_id": "UNKNOWN:0001",
  "term_label": "Unknown molecular function"
}